{
  "gene": "UniProtKB:Q9H4I8",
  "gene_name": "Serine hydrolase-like protein 2",
  "term_id": "UNKNOWN:0003",
  "gene_symbol": "SERHL2",
  "term_label": "Unknown cellular component"
}